{
  "term_label": "Unknown molecular function",
  "gene_symbol": "ATOSA",
  "gene": "UniProtKB:Q32MH5",
  "gene_name": "Atos homolog protein A",
  "term_id": "UNKNOWN:0001"
}